SUMO-specific endopeptidase activity [GO:0070139] (molecular function) Definition: Catalysis of the hydrolysis of peptide bonds between an alpha-carboxyl group and an alpha-amino group within the small conjugating protein SUMO. Sources: GOC:mah Relationships: is a type of ubiquitin-like protein-specific endopeptidase activity [GO:0070137]